{
  "gene_symbol": "TTC38",
  "gene_name": "Tetratricopeptide repeat protein 38",
  "term_label": "Unknown cellular component",
  "gene": "UniProtKB:Q5R3I4",
  "term_id": "UNKNOWN:0003"
}